{
  "gene_name": "Probable non-functional immunoglobulin heavy variable 1-38-4",
  "gene_symbol": "IGHV1-38-4",
  "term_label": "immunoglobulin mediated immune response",
  "term_id": "GO:0016064",
  "gene": "UniProtKB:P0DTW3"
}